aromatic desulfoglucosinolate sulfotransferase activity [GO:0047364] (MF) Sources: EC:2.8.2.24 Relationships: is a type of GO:0008146 Also known as: desulfoglucosinolate sulfotransferase activity, desulphoglucosinolate sulphotransferase activity, 3'-phosphoadenosine-5'-phosphosulfate:desulfoglucosinolate sulfotransferase activity, 3'-phosphoadenylyl-sulfate:desulfoglucosinolate sulfotransferase activity, PAPS-desulfoglucosinolate sulfotransferase activity Definition: Catalysis of the reaction: (Z)-desulfoglucotropeolin + 3'-phosphoadenylyl sulfate = (Z)-glucotropeolin + adenosine 3',5'-bisphosphate + H+. Also converts (Z)-indolylmethyl desulfoglucosinolate to (Z)-glucobrassicin. This is the final step in the biosynthesis of the glucosinolate core structure.